{
  "gene_symbol": "BMP6",
  "gene": "UniProtKB:P22004",
  "term_id": "GO:0007507",
  "gene_name": "Bone morphogenetic protein 6",
  "term_label": "heart development"
}